{
  "gene": "UniProtKB:Q9UL52",
  "term_label": "plasma membrane",
  "gene_symbol": "TMPRSS11E",
  "gene_name": "Transmembrane protease serine 11E",
  "term_id": "GO:0005886"
}